regulation of Schwann cell differentiation [GO:0014038] (BP) Subtypes: negative regulation of Schwann cell differentiation [GO:0014039], positive regulation of Schwann cell differentiation [GO:0014040] Relationships: is a type of regulation of glial cell differentiation [GO:0045685]; RO_0002211 Schwann cell differentiation [GO:0014037] Sources: GOC:ef Definition: Any process that modulates the frequency, rate or extent of Schwann cell differentiation.